{
  "gene_name": "E3 ubiquitin-protein ligase NHLRC1",
  "term_id": "GO:0043161",
  "term_label": "proteasome-mediated ubiquitin-dependent protein catabolic process",
  "gene": "UniProtKB:Q6VVB1",
  "gene_symbol": "NHLRC1"
}